{
  "gene_symbol": "RPAP2",
  "gene": "UniProtKB:Q8IXW5",
  "term_id": "GO:0008420",
  "gene_name": "Putative RNA polymerase II subunit B1 CTD phosphatase RPAP2",
  "term_label": "RNA polymerase II CTD heptapeptide repeat phosphatase activity"
}